{
  "term_id": "GO:0044853",
  "gene_symbol": "LYPD4",
  "term_label": "plasma membrane raft",
  "gene_name": "Ly6_PLAUR domain-containing protein 4",
  "gene": "UniProtKB:Q6UWN0"
}